DNA topoisomerase type I (single strand cut, ATP-independent) activity [GO:0003917] (MF) Definition: Catalysis of a DNA topological transformation by transiently cleaving one DNA strand at a time to allow passage of another strand; changes the linking number by +1 per catalytic cycle. Also known as: deoxyribonucleate topoisomerase, topoisomerase, type I DNA topoisomerase activity, type I topoisomerase activity, DNA topoisomerase I activity, nicking-closing enzyme activity, omega-protein activity, relaxing enzyme activity, swivelase activity, untwisting enzyme activity Relationships: is a type of DNA topoisomerase activity [GO:0003916] Note: Note that a further distinction, between type IA and type IB topoisomerases, is based on sequence or structural similarity between gene products that possess type I catalytic activity. References: PMID:8811192